{
  "term_id": "GO:0061631",
  "gene_name": "Ubiquitin-conjugating enzyme E2 D2",
  "gene": "UniProtKB:P62837",
  "gene_symbol": "UBE2D2",
  "term_label": "ubiquitin conjugating enzyme activity"
}